fibrillar collagen [GO:0098643] (cellular component) Relationships: is a type of GO:0098644; is part of GO:0140152 Definition: A supramolecular assembly of fibrillar collagen complexes in the form of a long fiber (fibril) with transverse striations (bands). References: PMID:20386646, PMID:21421911, PMID:29853175 Sources: GOC:dos Also known as: banded collagen fibril